proximal/distal pattern formation involved in metanephric nephron development [GO:0072272] (biological process) Relationships: is a type of proximal/distal pattern formation involved in nephron development [GO:0072047]; is a type of GO:0072268; is part of metanephric nephron development [GO:0072210] Sources: GOC:mtg_kidney_jan10 Also known as: proximal-distal pattern formation involved in metanephric nephron development, proximal/distal metanephric nephron patterning Definition: The regionalization process in which specific areas of cell differentiation are determined along a proximal/distal axis of a nephron in the metanephros. The proximal/distal axis is defined by a line that runs from the center of the kidney (proximal end) outward (distal end).